negative regulation of endoplasmic reticulum stress-induced intrinsic apoptotic signaling pathway [GO:1902236] (biological process) Also known as: down regulation of ER stress-induced apoptosis, down regulation of apoptosis in response to ER stress, down regulation of apoptosis triggered by ER stress, down regulation of endoplasmic reticulum stress-induced apoptosis, down regulation of intrinsic apoptotic signaling pathway in response to endoplasmic reticulum stress, down regulation of intrinsic apoptotic signaling pathway induced by endoplasmic reticulum stress, down-regulation of ER stress-induced apoptosis, down-regulation of apoptosis in response to ER stress, down-regulation of apoptosis triggered by ER stress, down-regulation of endoplasmic reticulum stress-induced apoptosis, down-regulation of intrinsic apoptotic signaling pathway in response to endoplasmic reticulum stress, down-regulation of intrinsic apoptotic signaling pathway induced by endoplasmic reticulum stress, downregulation of ER stress-induced apoptosis, downregulation of apoptosis in response to ER stress, downregulation of apoptosis triggered by ER stress, downregulation of endoplasmic reticulum stress-induced apoptosis, downregulation of intrinsic apoptotic signaling pathway in response to endoplasmic reticulum stress, downregulation of intrinsic apoptotic signaling pathway induced by endoplasmic reticulum stress, negative regulation of ER stress-induced apoptosis, negative regulation of apoptosis in response to ER stress, negative regulation of apoptosis triggered by ER stress, negative regulation of endoplasmic reticulum stress-induced apoptosis, negative regulation of intrinsic apoptotic signaling pathway in response to endoplasmic reticulum stress, negative regulation of intrinsic apoptotic signaling pathway induced by endoplasmic reticulum stress, inhibition of ER stress-induced apoptosis, inhibition of apoptosis in response to ER stress, inhibition of apoptosis triggered by ER stress, inhibition of endoplasmic reticulum stress-induced apoptosis, inhibition of intrinsic apoptotic signaling pathway in response to endoplasmic reticulum stress, inhibition of intrinsic apoptotic signaling pathway induced by endoplasmic reticulum stress Subtypes: negative regulation of endoplasmic reticulum stress-induced neuron intrinsic apoptotic signaling pathway [GO:1903382] Definition: Any process that stops, prevents or reduces the frequency, rate or extent of an endoplasmic reticulum stress-induced intrinsic apoptotic signaling pathway. Relationships: is a type of regulation of endoplasmic reticulum stress-induced intrinsic apoptotic signaling pathway [GO:1902235]; is a type of negative regulation of response to endoplasmic reticulum stress [GO:1903573]; is a type of negative regulation of intrinsic apoptotic signaling pathway [GO:2001243]; negatively regulates intrinsic apoptotic signaling pathway in response to endoplasmic reticulum stress [GO:0070059] References: PMID:20160352 Sources: GOC:BHF, GOC:TermGenie, GOC:mtg_apoptosis, GOC:rl